host cell surface [GO:0044228] (cellular component) Relationships: is a type of host cell part [GO:0033643] Definition: The external part of the host cell wall and/or host plasma membrane. Sources: GOC:rph